L-threonate 3-dehydrogenase activity [GO:0050036] (molecular function) Sources: EC:1.1.1.129, RHEA:23376 Relationships: is a type of oxidoreductase activity, acting on the CH-OH group of donors, NAD or NADP as acceptor [GO:0016616] Also known as: L-threonate:NAD+ 3-oxidoreductase activity, L-threonic acid dehydrogenase activity, threonate dehydrogenase activity Definition: Catalysis of the reaction: L-threonate + NAD+ = 3-dehydro-L-threonate + H+ + NADH.